{
  "term_label": "Unknown cellular component",
  "term_id": "UNKNOWN:0003",
  "gene": "UniProtKB:Q96A22",
  "gene_name": "Uncharacterized protein C11orf52",
  "gene_symbol": "C11orf52"
}